{
  "gene_name": "Uncharacterized protein",
  "gene": "UniProtKB:A0A494C030",
  "gene_symbol": "LOC114841035",
  "term_label": "Unknown molecular function",
  "term_id": "UNKNOWN:0001"
}